{
  "gene_name": "OTU domain-containing protein 4",
  "term_label": "negative regulation of toll-like receptor signaling pathway",
  "gene": "UniProtKB:Q01804",
  "gene_symbol": "OTUD4",
  "term_id": "GO:0034122"
}